{
  "gene_symbol": "CYP21A2",
  "gene_name": "Steroid 21-hydroxylase",
  "gene": "UniProtKB:P08686",
  "term_id": "GO:0020037",
  "term_label": "heme binding"
}